{
  "term_id": "GO:0030008",
  "gene_symbol": "TRAPPC3L",
  "gene": "UniProtKB:Q5T215",
  "gene_name": "Trafficking protein particle complex subunit 3-like protein",
  "term_label": "TRAPP complex"
}